{
  "gene_symbol": "ELMOD1",
  "gene_name": "ELMO domain-containing protein 1",
  "term_label": "GTPase activator activity",
  "term_id": "GO:0005096",
  "gene": "UniProtKB:Q8N336"
}